{
  "gene": "UniProtKB:P02042",
  "term_label": "erythrocyte development",
  "gene_symbol": "HBD",
  "term_id": "GO:0048821",
  "gene_name": "Hemoglobin subunit delta"
}